{
  "term_id": "GO:0005634",
  "gene_symbol": "NONO",
  "gene_name": "Non-POU domain-containing octamer-binding protein",
  "gene": "UniProtKB:Q15233",
  "term_label": "nucleus"
}